lateral motor column neuron migration [GO:0097477] (biological process) Relationships: is a type of GO:0097476 Regulation: regulated by regulation of lateral motor column neuron migration [GO:1902076]; negatively regulated by negative regulation of lateral motor column neuron migration [GO:1902077]; RO_0002213 by positive regulation of lateral motor column neuron migration [GO:1902078] Definition: The orderly movement of a lateral motor column neuron from one site to another. A lateral motor column neuron is a motor neuron that is generated only on limb levels and send axons into the limb mesenchyme. References: PMID:20711475 Sources: CL:0011002, GOC:yaf